{
  "gene": "UniProtKB:Q16877",
  "term_id": "GO:0003873",
  "gene_name": "6-phosphofructo-2-kinase_fructose-2,6-bisphosphatase 4",
  "gene_symbol": "PFKFB4",
  "term_label": "6-phosphofructo-2-kinase activity"
}